{
  "gene": "UniProtKB:P55199",
  "gene_name": "RNA polymerase II elongation factor ELL",
  "term_id": "GO:0008023",
  "gene_symbol": "ELL",
  "term_label": "transcription elongation factor complex"
}